{
  "term_id": "UNKNOWN:0001",
  "gene_name": "Zinc finger CCCH-type antiviral protein 1-like",
  "gene_symbol": "ZC3HAV1L",
  "gene": "UniProtKB:Q96H79",
  "term_label": "Unknown molecular function"
}